{
  "term_id": "UNKNOWN:0003",
  "gene_name": "Keratin-associated protein 10-8",
  "term_label": "Unknown cellular component",
  "gene": "UniProtKB:P60410",
  "gene_symbol": "KRTAP10-8"
}